{
  "gene_name": "E3 ubiquitin-protein ligase MARCHF3",
  "gene": "UniProtKB:Q86UD3",
  "term_id": "GO:0004842",
  "term_label": "ubiquitin-protein transferase activity",
  "gene_symbol": "MARCHF3"
}